{
  "gene": "UniProtKB:Q9H324",
  "gene_name": "A disintegrin and metalloproteinase with thrombospondin motifs 10",
  "term_label": "proteolysis",
  "term_id": "GO:0006508",
  "gene_symbol": "ADAMTS10"
}